lipid transport [GO:0006869] (biological process) Definition: The directed movement of lipids into, out of or within a cell, or between cells, by means of some agent such as a transporter or pore. Lipids are compounds soluble in an organic solvent but not, or sparingly, in an aqueous solvent. Sources: ISBN:0198506732 Relationships: is a type of transport [GO:0006810]; is part of lipid localization [GO:0010876] Regulation: regulated by regulation of lipid transport [GO:0032368]; negatively regulated by GO:0032369; positively regulated by positive regulation of lipid transport [GO:0032370] Subtypes: lipid antigen transport [GO:0002494], lipid transport involved in lipid storage [GO:0010877], GO:0015721, fatty acid transport [GO:0015908], GO:0015914, GO:0015918, lipopolysaccharide transport [GO:0015920], intracellular lipid transport [GO:0032365], acylglycerol transport [GO:0034196], lipid translocation [GO:0034204], GO:0035627, polymyxin transport [GO:0042893], glycolipid transport [GO:0046836], GO:0046864, intermembrane lipid transfer [GO:0120009], lipid export from cell [GO:0140353], lipid import into cell [GO:0140354], lipid hydroperoxide transport [GO:1901373], GO:1901571, sphingoid long-chain base transport [GO:1905329], lipid transport across blood-brain barrier [GO:1990379]